cytoplasm organization [GO:0007028] (biological process) Definition: A process that is carried out at the cellular level which results in the assembly, arrangement of constituent parts, or disassembly of the cytoplasm. The cytoplasm is all of the contents of a cell excluding the plasma membrane and nucleus, but including other subcellular structures. Sources: GOC:curators, GOC:dph, GOC:jl, GOC:mah Also known as: cytoplasm organisation, cytoplasm organization and biogenesis Relationships: is a type of cellular component organization [GO:0016043] Subtypes: vitellogenesis [GO:0007296], GO:0007315